{
  "gene_symbol": "AFAP1",
  "gene_name": "Actin filament-associated protein 1",
  "term_label": "Unknown molecular function",
  "term_id": "UNKNOWN:0001",
  "gene": "UniProtKB:Q8N556"
}